cell wall organization involved in conjugation with cellular fusion [GO:0070871] (biological process) Definition: A process of cell wall organization that contributes to conjugation with cellular fusion. Relationships: is a type of cell wall organization [GO:0071555]; is part of GO:0000747 Also known as: cell wall organisation involved in conjugation with cellular fusion Sources: GOC:mah Subtypes: fungal-type cell wall disassembly involved in conjugation with cellular fusion [GO:1904541]